negative regulation of polynucleotide adenylyltransferase activity [GO:1904246] (biological process) Also known as: down regulation of AMP polynucleotidylexotransferase activity, down regulation of ATP-polynucleotide adenylyltransferase activity, down regulation of ATP:polynucleotide adenylyltransferase activity, down regulation of ATP:polynucleotidylexotransferase activity, down regulation of NTP polymerase activity, down regulation of RNA adenylating enzyme activity, down regulation of adenosine triphosphate:ribonucleic acid adenylyltransferase activity, down regulation of poly(A) hydrolase activity, down regulation of poly(A) polymerase activity, down regulation of poly(A) synthetase activity, down regulation of poly-A polymerase activity, down regulation of polyadenylate nucleotidyltransferase activity, down regulation of polyadenylate polymerase activity, down regulation of polyadenylate synthetase activity, down regulation of polyadenylic acid polymerase activity, down regulation of polyadenylic polymerase activity, down regulation of polynucleotide adenylyltransferase activity, down regulation of terminal riboadenylate transferase activity, down-regulation of AMP polynucleotidylexotransferase activity, down-regulation of ATP-polynucleotide adenylyltransferase activity, down-regulation of ATP:polynucleotide adenylyltransferase activity, down-regulation of ATP:polynucleotidylexotransferase activity, down-regulation of NTP polymerase activity, down-regulation of RNA adenylating enzyme activity, down-regulation of adenosine triphosphate:ribonucleic acid adenylyltransferase activity, down-regulation of poly(A) hydrolase activity, down-regulation of poly(A) polymerase activity, down-regulation of poly(A) synthetase activity, down-regulation of poly-A polymerase activity, down-regulation of polyadenylate nucleotidyltransferase activity, down-regulation of polyadenylate polymerase activity, down-regulation of polyadenylate synthetase activity, down-regulation of polyadenylic acid polymerase activity, down-regulation of polyadenylic polymerase activity, down-regulation of polynucleotide adenylyltransferase activity, down-regulation of terminal riboadenylate transferase activity, downregulation of AMP polynucleotidylexotransferase activity, downregulation of ATP-polynucleotide adenylyltransferase activity, downregulation of ATP:polynucleotide adenylyltransferase activity, downregulation of ATP:polynucleotidylexotransferase activity, downregulation of NTP polymerase activity, downregulation of RNA adenylating enzyme activity, downregulation of adenosine triphosphate:ribonucleic acid adenylyltransferase activity, downregulation of poly(A) hydrolase activity, downregulation of poly(A) polymerase activity, downregulation of poly(A) synthetase activity, downregulation of poly-A polymerase activity, downregulation of polyadenylate nucleotidyltransferase activity, downregulation of polyadenylate polymerase activity, downregulation of polyadenylate synthetase activity, downregulation of polyadenylic acid polymerase activity, downregulation of polyadenylic polymerase activity, downregulation of polynucleotide adenylyltransferase activity, downregulation of terminal riboadenylate transferase activity, negative regulation of AMP polynucleotidylexotransferase activity, negative regulation of ATP-polynucleotide adenylyltransferase activity, negative regulation of ATP:polynucleotide adenylyltransferase activity, negative regulation of ATP:polynucleotidylexotransferase activity, negative regulation of NTP polymerase activity, negative regulation of RNA adenylating enzyme activity, negative regulation of adenosine triphosphate:ribonucleic acid adenylyltransferase activity, negative regulation of poly(A) hydrolase activity, negative regulation of poly(A) polymerase activity, negative regulation of poly(A) synthetase activity, negative regulation of poly-A polymerase activity, negative regulation of polyadenylate nucleotidyltransferase activity, negative regulation of polyadenylate polymerase activity, negative regulation of polyadenylate synthetase activity, negative regulation of polyadenylic acid polymerase activity, negative regulation of polyadenylic polymerase activity, negative regulation of terminal riboadenylate transferase activity, inhibition of AMP polynucleotidylexotransferase activity, inhibition of ATP-polynucleotide adenylyltransferase activity, inhibition of ATP:polynucleotide adenylyltransferase activity, inhibition of ATP:polynucleotidylexotransferase activity, inhibition of NTP polymerase activity, inhibition of RNA adenylating enzyme activity, inhibition of adenosine triphosphate:ribonucleic acid adenylyltransferase activity, inhibition of poly(A) hydrolase activity, inhibition of poly(A) polymerase activity, inhibition of poly(A) synthetase activity, inhibition of poly-A polymerase activity, inhibition of polyadenylate nucleotidyltransferase activity, inhibition of polyadenylate polymerase activity, inhibition of polyadenylate synthetase activity, inhibition of polyadenylic acid polymerase activity, inhibition of polyadenylic polymerase activity, inhibition of polynucleotide adenylyltransferase activity, inhibition of terminal riboadenylate transferase activity, down regulation of RNA formation factors, PF1, down-regulation of RNA formation factors, PF1, downregulation of RNA formation factors, PF1, inhibition of RNA formation factors, PF1, negative regulation of RNA formation factors, PF1 Definition: Any process that stops, prevents or reduces the frequency, rate or extent of polynucleotide adenylyltransferase activity. References: PMID:19460348 Sources: GOC:TermGenie, GOC:kmv, GO_REF:0000059 Relationships: is a type of GO:0043086; is a type of regulation of transferase activity [GO:0051338]; negatively regulates poly(A) RNA polymerase activity [GO:1990817]